regulation of dendritic cell differentiation [GO:2001198] (biological process) Subtypes: negative regulation of dendritic cell differentiation [GO:2001199], positive regulation of dendritic cell differentiation [GO:2001200] Definition: Any process that modulates the frequency, rate or extent of dendritic cell differentiation. Relationships: is a type of regulation of leukocyte differentiation [GO:1902105]; regulates GO:0097028 Sources: GOC:obol